{
  "gene": "UniProtKB:Q8TDF6",
  "term_id": "GO:0007265",
  "term_label": "Ras protein signal transduction",
  "gene_name": "RAS guanyl-releasing protein 4",
  "gene_symbol": "RASGRP4"
}